{
  "gene_symbol": "IGF2BP3",
  "gene_name": "Insulin-like growth factor 2 mRNA-binding protein 3",
  "gene": "UniProtKB:O00425",
  "term_label": "cytoplasm",
  "term_id": "GO:0005737"
}